2-hydroxycyclohexanone 2-monooxygenase activity [GO:0047095] (molecular function) Sources: EC:1.14.13.66, RHEA:33283 Also known as: 2-hydroxycyclohexan-1-one,NADPH:oxygen 2-oxidoreductase (1,2-lactonizing) Relationships: is a type of oxidoreductase activity, acting on paired donors, with incorporation or reduction of molecular oxygen, NAD(P)H as one donor, and incorporation of one atom of oxygen [GO:0016709] Definition: Catalysis of the reaction: 2-hydroxycyclohexan-1-one + NADPH + O2 = 6-oxohexanoate + H2O + NADP+.